{
  "gene_symbol": "SCML4",
  "term_label": "negative regulation of DNA-templated transcription",
  "term_id": "GO:0045892",
  "gene_name": "Sex comb on midleg-like protein 4",
  "gene": "UniProtKB:Q8N228"
}